{
  "term_id": "UNKNOWN:0003",
  "gene": "UniProtKB:Q9NZP5",
  "term_label": "Unknown cellular component",
  "gene_name": "Olfactory receptor 5AC2",
  "gene_symbol": "OR5AC2"
}